{
  "gene": "UniProtKB:Q9Y5S8",
  "gene_name": "NADPH oxidase 1",
  "term_id": "GO:0006952",
  "term_label": "defense response",
  "gene_symbol": "NOX1"
}